{
  "term_id": "UNKNOWN:0001",
  "gene_symbol": "ZC2HC1A",
  "gene": "UniProtKB:Q96GY0",
  "term_label": "Unknown molecular function",
  "gene_name": "Zinc finger C2HC domain-containing protein 1A"
}